epithelial cell differentiation involved in mammary gland cord morphogenesis [GO:0060653] (biological process) Relationships: is_a mammary gland epithelial cell differentiation [GO:0060644]; is part of mammary gland cord morphogenesis [GO:0060652] Definition: The process in which a relatively unspecialized epithelial cell becomes a more specialized epithelial cell of the mammary gland cord. Epithelial cells of the mammary cord give it its funnel-like shape and some are cornified. Also known as: epithelial cell differentiation involved in mammary gland sprout morphogenesis References: PMID:12558599 Sources: GOC:dph